{
  "term_label": "actin filament binding",
  "gene": "UniProtKB:Q9ULV4",
  "gene_name": "Coronin-1C",
  "term_id": "GO:0051015",
  "gene_symbol": "CORO1C"
}